{
  "gene_name": "Retinal guanylyl cyclase 2",
  "term_id": "GO:0004383",
  "term_label": "guanylate cyclase activity",
  "gene": "UniProtKB:P51841",
  "gene_symbol": "GUCY2F"
}